positive regulation of calcium import into the mitochondrion [GO:0110098] (biological process) Definition: Any process that activates or increases the frequency, rate or extent of calcium import into the mitochondrion. References: PMID:24085037 Sources: GOC:sl Relationships: is a type of regulation of calcium import into the mitochondrion [GO:0110097]; is a type of positive regulation of calcium ion transmembrane transport [GO:1904427]; positively regulates calcium import into the mitochondrion [GO:0036444]